{
  "term_id": "GO:0005886",
  "term_label": "plasma membrane",
  "gene": "UniProtKB:Q13241",
  "gene_symbol": "KLRD1",
  "gene_name": "Natural killer cells antigen CD94"
}